response to immobilization stress combined with electrical stimulus [GO:1990781] (biological process) References: PMID:17008368 Relationships: is a type of response to immobilization stress [GO:0035902]; is a type of response to electrical stimulus [GO:0051602] Definition: Any process that results in a change in state or activity of a cell or an organism (in terms of movement, secretion, enzyme production, gene expression, etc.) as a result of an electrical stimulus given while being held immobile.